{
  "term_label": "extracellular space",
  "gene_name": "Histone H2B type 3-B",
  "term_id": "GO:0005615",
  "gene_symbol": "H2BC26",
  "gene": "UniProtKB:Q8N257"
}